{
  "gene_symbol": "ZNF85",
  "term_id": "GO:0000981",
  "gene_name": "Zinc finger protein 85",
  "term_label": "DNA-binding transcription factor activity, RNA polymerase II-specific",
  "gene": "UniProtKB:Q03923"
}